{
  "gene": "UniProtKB:P11168",
  "gene_name": "Solute carrier family 2, facilitated glucose transporter member 2",
  "term_id": "GO:0046323",
  "term_label": "D-glucose import",
  "gene_symbol": "SLC2A2"
}